{
  "gene": "UniProtKB:O14733",
  "term_label": "stress-activated MAPK cascade",
  "term_id": "GO:0051403",
  "gene_symbol": "MAP2K7",
  "gene_name": "Dual specificity mitogen-activated protein kinase kinase 7"
}